{
  "term_label": "axonemal central apparatus",
  "gene": "UniProtKB:Q6Q759",
  "gene_symbol": "SPAG17",
  "gene_name": "Sperm-associated antigen 17",
  "term_id": "GO:1990716"
}